{
  "gene_symbol": "HTR1B",
  "term_label": "G protein-coupled receptor signaling pathway, coupled to cyclic nucleotide second messenger",
  "term_id": "GO:0007187",
  "gene_name": "5-hydroxytryptamine receptor 1B",
  "gene": "UniProtKB:P28222"
}